{
  "term_label": "microtubule-based movement",
  "gene_name": "Dynein light chain roadblock-type 2",
  "gene": "UniProtKB:Q8TF09",
  "gene_symbol": "DYNLRB2",
  "term_id": "GO:0007018"
}